{
  "gene_name": "Solute carrier family 12 member 4",
  "term_label": "plasma membrane",
  "gene_symbol": "SLC12A4",
  "gene": "UniProtKB:Q9UP95",
  "term_id": "GO:0005886"
}